{
  "term_id": "UNKNOWN:0001",
  "gene": "UniProtKB:Q5HYL7",
  "gene_symbol": "TMEM196",
  "gene_name": "Transmembrane protein 196",
  "term_label": "Unknown molecular function"
}